regulation of smoothened signaling pathway involved in dorsal/ventral neural tube patterning [GO:1901620] (biological process) Sources: GOC:TermGenie Subtypes: GO:1901621, positive regulation of smoothened signaling pathway involved in dorsal/ventral neural tube patterning [GO:1901622] Also known as: regulation of hedgehog signaling pathway involved in dorsal/ventral neural tube patterning, regulation of hh signaling pathway involved in dorsal/ventral neural tube patterning, regulation of smoothened signalling pathway involved in dorsal/ventral neural tube patterning Relationships: is a type of regulation of smoothened signaling pathway [GO:0008589]; regulates smoothened signaling pathway involved in dorsal/ventral neural tube patterning [GO:0060831] Definition: Any process that modulates the frequency, rate or extent of smoothened signaling pathway involved in dorsal/ventral neural tube patterning.